ent-pimara-8(14),15-diene biosynthetic process [GO:1901541] (biological process) Regulation: regulated by regulation of ent-pimara-8(14),15-diene biosynthetic process [GO:1901542]; negatively regulated by negative regulation of ent-pimara-8(14),15-diene biosynthetic process [GO:1901543]; positively regulated by positive regulation of ent-pimara-8(14),15-diene biosynthetic process [GO:1901544] Relationships: is a type of terpene biosynthetic process [GO:0046246] Definition: The chemical reactions and pathways resulting in the formation of ent-pimara-8(14),15-diene. Sources: GOC:TermGenie, GOC:di Also known as: ent-pimara-8(14),15-diene anabolism, ent-pimara-8(14),15-diene biosynthesis, ent-pimara-8(14),15-diene formation, ent-pimara-8(14),15-diene synthesis